{
  "gene_symbol": "CCT6A",
  "gene": "UniProtKB:P40227",
  "term_label": "chaperonin-containing T-complex",
  "term_id": "GO:0005832",
  "gene_name": "T-complex protein 1 subunit zeta"
}